{
  "term_id": "GO:0005829",
  "gene_name": "Serine_threonine-protein kinase D1",
  "gene_symbol": "PRKD1",
  "term_label": "cytosol",
  "gene": "UniProtKB:Q15139"
}